{
  "gene": "UniProtKB:Q9H1R2",
  "gene_symbol": "DUSP15",
  "term_label": "positive regulation of ERK1 and ERK2 cascade",
  "gene_name": "Dual specificity protein phosphatase 15",
  "term_id": "GO:0070374"
}